peptide transport [GO:0015833] (biological process) Subtypes: peptide secretion [GO:0002790], oligopeptide transport [GO:0006857], peptidoglycan-associated peptide transport [GO:0015834], peptide antigen transport [GO:0046968], dipeptide transmembrane transport from lysosomal lumen to cytosol [GO:0141204] Relationships: is a type of amide transport [GO:0042886] Sources: GOC:ai Definition: The directed movement of peptides, compounds of two or more amino acids where the alpha carboxyl group of one is bound to the alpha amino group of another, into, out of or within a cell, or between cells, by means of some agent such as a transporter or pore. Regulation: regulated by regulation of peptide transport [GO:0090087]